{
  "gene_name": "2-Hydroxyacid oxidase 2",
  "term_label": "peroxisomal matrix",
  "gene_symbol": "HAO2",
  "term_id": "GO:0005782",
  "gene": "UniProtKB:Q9NYQ3"
}